organellar small ribosomal subunit [GO:0000314] (CC) Relationships: is a type of small ribosomal subunit [GO:0015935]; is part of organellar ribosome [GO:0000313] Definition: The smaller of the two subunits of an organellar ribosome. Subtypes: GO:0000312, mitochondrial small ribosomal subunit [GO:0005763] Sources: GOC:mcc